{
  "gene": "UniProtKB:P29466",
  "gene_symbol": "CASP1",
  "gene_name": "Caspase-1",
  "term_id": "GO:0016485",
  "term_label": "protein processing"
}